{
  "gene": "UniProtKB:P52888",
  "gene_name": "Thimet oligopeptidase",
  "term_label": "mitochondrial intermembrane space",
  "term_id": "GO:0005758",
  "gene_symbol": "THOP1"
}